{
  "gene_symbol": "TOX2",
  "term_label": "regulation of transcription by RNA polymerase II",
  "gene_name": "TOX high mobility group box family member 2",
  "gene": "UniProtKB:Q96NM4",
  "term_id": "GO:0006357"
}